{
  "term_id": "GO:0006357",
  "gene": "UniProtKB:P0CG23",
  "term_label": "regulation of transcription by RNA polymerase II",
  "gene_symbol": "ZNF853",
  "gene_name": "Zinc finger protein 853"
}